{
  "gene_name": "Osteoclast stimulatory transmembrane protein",
  "gene_symbol": "OCSTAMP",
  "gene": "UniProtKB:Q9BR26",
  "term_label": "Unknown biological process",
  "term_id": "UNKNOWN:0002"
}